noradrenergic neuron development [GO:0003358] (biological process) Relationships: is a type of neuron development [GO:0048666]; is part of noradrenergic neuron differentiation [GO:0003357] Definition: The process whose specific outcome is the progression of a noradrenergic neuron over time, from initial commitment of the cell to a specific fate, to the fully functional differentiated cell. Sources: GOC:dph Also known as: norepinephrine secreting neuron development